regulation of cardiac muscle myoblast proliferation [GO:0110022] (biological process) Relationships: is_a regulation of myoblast proliferation [GO:2000291]; regulates cardiac muscle myoblast proliferation [GO:0110021] References: PMID:26512644 Sources: GOC:BHF, GOC:BHF_miRNA, GOC:rph Definition: Any process that modulates the frequency, rate or extent of cardiac muscle myoblast proliferation. Subtypes: negative regulation of cardiac muscle myoblast proliferation [GO:0110023], positive regulation of cardiac muscle myoblast proliferation [GO:0110024]